neural plate development [GO:0001840] (biological process) Sources: GOC:dph, GOC:ef, ISBN:0878932437, ISBN:0878932585 Definition: The process whose specific outcome is the progression of the neural plate over time, from its formation to the mature structure. The neural plate is a flat, thickened layer of ectodermal cells. The underlying dorsal mesoderm signals the ectodermal cells above it to elongate into columnar neural plate cells. The neural plate subsequently develops into the neural tube, which gives rise to the central nervous system. Relationships: is a type of epithelium development [GO:0060429]; is part of chordate embryonic development [GO:0043009]